{
  "gene_name": "Disintegrin and metalloproteinase domain-containing protein 2",
  "gene": "UniProtKB:Q99965",
  "term_id": "GO:0007155",
  "term_label": "cell adhesion",
  "gene_symbol": "ADAM2"
}